negative regulation of TORC2 signaling [GO:1903940] (biological process) Relationships: is a type of negative regulation of TOR signaling [GO:0032007]; is a type of regulation of TORC2 signaling [GO:1903939]; negatively regulates GO:0038203 References: PMID:24247430 Sources: GOC:TermGenie, GO_REF:0000058 Definition: Any process that stops, prevents or reduces the frequency, rate or extent of TORC2 signaling. Also known as: down regulation of TORC2 signal transduction, down regulation of TORC2 signaling, down-regulation of TORC2 signal transduction, down-regulation of TORC2 signaling, downregulation of TORC2 signal transduction, downregulation of TORC2 signaling, negative regulation of TORC2 signal transduction, inhibition of TORC2 signal transduction, inhibition of TORC2 signaling